erythropoietin-mediated signaling pathway [GO:0038162] (biological process) Relationships: is_a cytokine-mediated signaling pathway [GO:0019221]; is part of GO:0036018 Also known as: EPO-R signaling pathway, erythropoietin receptor signaling pathway References: PMID:12489509 Sources: GOC:nhn Definition: The series of molecular signals initiated by erythropoietin (EPO) binding to the erythropoietin receptor (EPO-R) on the surface of a target cell, and ending with the regulation of a downstream cellular process, e.g. transcription.